{
  "gene_symbol": "COL19A1",
  "gene_name": "Collagen alpha-1(XIX) chain",
  "term_id": "GO:0030020",
  "term_label": "extracellular matrix structural constituent conferring tensile strength",
  "gene": "UniProtKB:Q14993"
}